negative regulation of ureter smooth muscle cell differentiation [GO:2000062] (biological process) Sources: GOC:mtg_kidney_jan10, GOC:obol, GOC:yaf Relationships: is a type of GO:0051151; is a type of negative regulation of multicellular organismal process [GO:0051241]; is a type of regulation of ureter smooth muscle cell differentiation [GO:2000061]; negatively regulates GO:0072193 Definition: Any process that stops, prevents, or reduces the frequency, rate or extent of ureter smooth muscle cell differentiation.